{
  "gene_symbol": "ADCY3",
  "gene_name": "Adenylate cyclase type 3",
  "term_label": "plasma membrane",
  "gene": "UniProtKB:O60266",
  "term_id": "GO:0005886"
}